diferuloyl mono-(hydroxyferuloyl) spermidine meta-hydroxylase activity [GO:0072551] (molecular function) Relationships: is a type of tri-(feruloyl or hydroxyferuloyl) spermidine meta-hydroxylase activity [GO:0072532] Definition: Catalysis of the reaction: diferuloyl mono-(hydroxyferuloyl) spermidine + NADPH + O2 = monoferuloyl di-(hydroxyferuloyl) spermidine + NADP+ + H2O. References: PMID:19779199 Sources: GOC:kad